{
  "term_id": "GO:0005737",
  "gene_name": "Serine_threonine-protein phosphatase 2A 65 kDa regulatory subunit A beta isoform",
  "gene_symbol": "PPP2R1B",
  "term_label": "cytoplasm",
  "gene": "UniProtKB:P30154"
}